{
  "term_id": "GO:0048194",
  "gene": "UniProtKB:Q9H4A5",
  "term_label": "Golgi vesicle budding",
  "gene_name": "Golgi phosphoprotein 3-like",
  "gene_symbol": "GOLPH3L"
}